{
  "gene_symbol": "JMJD7",
  "gene_name": "Bifunctional peptidase and (3S)-lysyl hydroxylase JMJD7",
  "gene": "UniProtKB:P0C870",
  "term_label": "endopeptidase activity",
  "term_id": "GO:0004175"
}